{
  "gene": "UniProtKB:Q8NHM5",
  "gene_symbol": "KDM2B",
  "gene_name": "Lysine-specific demethylase 2B",
  "term_id": "GO:0003712",
  "term_label": "transcription coregulator activity"
}